neuromuscular process controlling balance [GO:0050885] (biological process) Also known as: regulation of balance Relationships: is a type of neuromuscular process [GO:0050905]; BFO_0000051 musculoskeletal movement [GO:0050881] Sources: GOC:ai, GOC:dph Definition: Any process that an organism uses to control its balance, the orientation of the organism (or the head of the organism) in relation to the source of gravity. In humans and animals, balance is perceived through visual cues, the labyrinth system of the inner ears and information from skin pressure receptors and muscle and joint receptors.